{
  "term_id": "GO:0005759",
  "term_label": "mitochondrial matrix",
  "gene_name": "Presequence protease, mitochondrial",
  "gene": "UniProtKB:Q5JRX3",
  "gene_symbol": "PITRM1"
}